{
  "gene": "UniProtKB:Q9HBG7",
  "gene_symbol": "LY9",
  "term_label": "Unknown molecular function",
  "gene_name": "T-lymphocyte surface antigen Ly-9",
  "term_id": "UNKNOWN:0001"
}